{
  "gene_symbol": "DECR2",
  "term_id": "GO:0005777",
  "gene": "UniProtKB:Q9NUI1",
  "gene_name": "Peroxisomal 2,4-dienoyl-CoA reductase [(3E)-enoyl-CoA-producing]",
  "term_label": "peroxisome"
}